{
  "gene": "UniProtKB:A4D263",
  "gene_symbol": "SPMIP7",
  "gene_name": "Spermatogenesis-associated protein 48",
  "term_id": "UNKNOWN:0001",
  "term_label": "Unknown molecular function"
}